colneleate synthase activity [GO:0102895] (molecular function) Sources: EC:4.2.1.121, GOC:pz Definition: Catalysis of the reaction: 9(S)-HPODE = colneleate + H2O. Relationships: is a type of hydro-lyase activity [GO:0016836]